{
  "term_id": "GO:0000287",
  "gene_symbol": "CIB1",
  "gene": "UniProtKB:Q99828",
  "gene_name": "Calcium and integrin-binding protein 1",
  "term_label": "magnesium ion binding"
}